positive regulation of endocardial cushion to mesenchymal transition [GO:0140051] (biological process) Relationships: is a type of positive regulation of cardiac epithelial to mesenchymal transition [GO:0062043]; is a type of regulation of endocardial cushion to mesenchymal transition [GO:0140049]; positively regulates endocardial cushion to mesenchymal transition [GO:0090500] Subtypes: positive regulation of endocardial cushion to mesenchymal transition involved in heart valve formation [GO:2000802] References: PMID:21778427 Sources: GOC:BHF, GOC:BHF_miRNA, GOC:rph Definition: Any process that activates or increases the frequency, rate or extent of endocardial cushion to mesenchymal transition.